{
  "gene_name": "Lariat debranching enzyme",
  "term_label": "nucleus",
  "term_id": "GO:0005634",
  "gene_symbol": "DBR1",
  "gene": "UniProtKB:Q9UK59"
}